{
  "gene_symbol": "MIF",
  "gene_name": "Macrophage migration inhibitory factor",
  "term_label": "Unknown biological process",
  "term_id": "UNKNOWN:0002",
  "gene": "UniProtKB:P14174"
}